{
  "term_label": "extracellular matrix",
  "gene": "UniProtKB:Q99969",
  "gene_name": "Retinoic acid receptor responder protein 2",
  "gene_symbol": "RARRES2",
  "term_id": "GO:0031012"
}